{
  "gene_symbol": "TRPV3",
  "term_label": "plasma membrane",
  "gene_name": "Transient receptor potential cation channel subfamily V member 3",
  "gene": "UniProtKB:Q8NET8",
  "term_id": "GO:0005886"
}